6-alpha-maltosylglucose catabolic process [GO:0051681] (biological process) Sources: GOC:ai Also known as: isopanose catabolic process, isopanose catabolism Relationships: is a type of GO:0009313 Definition: The chemical reactions and pathways resulting in the breakdown of 6-alpha-maltosylglucose, also known as isopanose.